{
  "gene_symbol": "ZSCAN5C",
  "gene_name": "Zinc finger and SCAN domain-containing protein 5C",
  "term_label": "Unknown cellular component",
  "gene": "UniProtKB:A6NGD5",
  "term_id": "UNKNOWN:0003"
}